carbapenem catabolic process [GO:1901768] (biological process) Definition: The chemical reactions and pathways resulting in the breakdown of carbapenem. References: PMID:9402024 Sources: GOC:TermGenie, GOC:yaf Also known as: carbapenem breakdown, carbapenem catabolism, carbapenem degradation Relationships: is a type of beta-lactam antibiotic catabolic process [GO:0030655]